{
  "term_id": "UNKNOWN:0001",
  "gene_symbol": "EMP1",
  "gene": "UniProtKB:P54849",
  "term_label": "Unknown molecular function",
  "gene_name": "Epithelial membrane protein 1"
}